{
  "gene": "UniProtKB:Q8IYV9",
  "term_id": "GO:0007342",
  "gene_symbol": "IZUMO1",
  "term_label": "fusion of sperm to egg plasma membrane involved in single fertilization",
  "gene_name": "Izumo sperm-egg fusion protein 1"
}